{
  "gene": "UniProtKB:Q9Y6E0",
  "gene_symbol": "STK24",
  "gene_name": "Serine_threonine-protein kinase 24",
  "term_id": "GO:0004674",
  "term_label": "protein serine/threonine kinase activity"
}